{
  "term_id": "GO:0044715",
  "term_label": "8-oxo-dGDP phosphatase activity",
  "gene_name": "8-oxo-dGDP phosphatase NUDT18",
  "gene_symbol": "NUDT18",
  "gene": "UniProtKB:Q6ZVK8"
}